ent-pimara-9(11),15-diene synthase activity [GO:0052674] (MF) Sources: RHEA:25544 Also known as: PMD synthase activity, ent-copalyl-diphosphate diphosphate-lyase [ent-pimara-9(11),15-diene-forming] activity Relationships: is_a GO:0016838 Definition: Catalysis of the reaction: ent-copalyl diphosphate = ent-pimara-9(11),15-diene + diphosphate.